ribonucleotide catabolic process [GO:0009261] (biological process) Definition: The chemical reactions and pathways resulting in the breakdown of a ribonucleotide, a compound consisting of ribonucleoside (a base linked to a ribose sugar) esterified with a phosphate group at either the 3' or 5'-hydroxyl group of the sugar. Sources: GOC:go_curators, ISBN:0198506732 Subtypes: GO:0009154, pyrimidine ribonucleotide catabolic process [GO:0009222], FMN catabolic process [GO:0032363] Relationships: is a type of nucleotide catabolic process [GO:0009166]; is a type of ribonucleotide metabolic process [GO:0009259]; is a type of carbohydrate derivative catabolic process [GO:1901136] Also known as: ribonucleotide breakdown, ribonucleotide catabolism, ribonucleotide degradation